{
  "gene": "UniProtKB:P08048",
  "gene_symbol": "ZFY",
  "term_id": "GO:0006357",
  "term_label": "regulation of transcription by RNA polymerase II",
  "gene_name": "Zinc finger Y-chromosomal protein"
}